{
  "gene_symbol": "SLC32A1",
  "term_id": "GO:0044306",
  "gene_name": "Vesicular inhibitory amino acid transporter",
  "gene": "UniProtKB:Q9H598",
  "term_label": "neuron projection terminus"
}